{
  "gene_name": "Microtubule-associated protein 2",
  "gene": "UniProtKB:P11137",
  "gene_symbol": "MAP2",
  "term_label": "neuron projection development",
  "term_id": "GO:0031175"
}